renal capsule specification [GO:0072130] (biological process) Sources: GOC:mtg_kidney_jan10 Subtypes: mesonephric capsule specification [GO:0061288], metanephric capsule specification [GO:0072267] Relationships: is a type of regionalization [GO:0003002]; is a type of pattern specification involved in kidney development [GO:0061004]; is part of renal capsule formation [GO:0072129] Definition: The regionalization process in which the identity of the renal capsule is specified. Identity is considered to be the aggregate of characteristics by which a structure is recognized.